{
  "gene": "UniProtKB:P29084",
  "gene_symbol": "GTF2E2",
  "term_id": "GO:0005673",
  "term_label": "transcription factor TFIIE complex",
  "gene_name": "Transcription initiation factor IIE subunit beta"
}